{
  "gene_symbol": "LYSET",
  "term_id": "UNKNOWN:0002",
  "term_label": "Unknown biological process",
  "gene_name": "Lysosomal enzyme trafficking factor",
  "gene": "UniProtKB:Q8N6I4"
}